{
  "term_label": "innate immune response",
  "gene_symbol": "CLEC7A",
  "gene_name": "C-type lectin domain family 7 member A",
  "gene": "UniProtKB:Q9BXN2",
  "term_id": "GO:0045087"
}